[phosphorylase] phosphatase activity [GO:0050196] (MF) Relationships: is a type of GO:0004721 Sources: EC:3.1.3.17, MetaCyc:PHOSPHORYLASE-PHOSPHATASE-RXN Also known as: phosphorylase phosphatase activity, PR-enzyme, glycogen phosphorylase phosphatase activity, phosphorylase a phosphatase activity, phosphorylase a phosphohydrolase activity, protein phosphatase C, type 1 protein phosphatase activity Definition: Catalysis of the reaction: [phosphorylase a] + 4 H2O = 2 [phosphorylase b] + 4 phosphate.